negative regulation of butyryl-CoA biosynthetic process from acetyl-CoA [GO:1900495] (biological process) Definition: Any process that stops, prevents or reduces the frequency, rate or extent of butyryl-CoA biosynthetic process from acetyl-CoA. Sources: GOC:TermGenie, GOC:mengo_curators Relationships: is a type of negative regulation of amide metabolic process [GO:0034249]; is a type of negative regulation of fatty acid biosynthetic process [GO:0045717]; is_a negative regulation of nucleobase-containing compound metabolic process [GO:0045934]; is_a negative regulation of phosphate metabolic process [GO:0045936]; is a type of regulation of butyryl-CoA biosynthetic process from acetyl-CoA [GO:1900494]; negatively regulates butyryl-CoA biosynthetic process from acetyl-CoA [GO:0044579] Also known as: down regulation of butyryl-CoA biosynthesis from acetyl-CoA, down regulation of butyryl-CoA biosynthetic process from acetyl-CoA, down-regulation of butyryl-CoA biosynthesis from acetyl-CoA, down-regulation of butyryl-CoA biosynthetic process from acetyl-CoA, downregulation of butyryl-CoA biosynthesis from acetyl-CoA, downregulation of butyryl-CoA biosynthetic process from acetyl-CoA, inhibition of butyryl-CoA biosynthesis from acetyl-CoA, negative regulation of butyryl-CoA biosynthesis from acetyl-CoA, inhibition of butyryl-CoA biosynthetic process from acetyl-CoA